{
  "term_id": "GO:0099503",
  "gene_symbol": "BAIAP3",
  "gene_name": "BAI1-associated protein 3",
  "term_label": "secretory vesicle",
  "gene": "UniProtKB:O94812"
}